regulation of (1->6)-beta-D-glucan biosynthetic process [GO:0060917] (biological process) Relationships: is_a regulation of beta-glucan biosynthetic process [GO:0032951]; regulates (1->6)-beta-D-glucan biosynthetic process [GO:0006078] Definition: Any process that modulates the frequency, rate or extent of the chemical reactions and pathways resulting in the formation of (1->6)-beta-D-glucans. Also known as: regulation of 1,6-beta-glucan biosynthetic process Sources: GOC:dph, GOC:tb